positive regulation of autophagosome size [GO:0045772] (biological process) Sources: GOC:autophagy, GOC:go_curators Also known as: positive regulation of autophagic vacuole size, up regulation of autophagic vacuole size, up-regulation of autophagic vacuole size, upregulation of autophagic vacuole size, activation of autophagic vacuole size, stimulation of autophagic vacuole size Definition: Any process that increases autophagosome size. Relationships: is a type of regulation of autophagosome size [GO:0016243]